histone pre-mRNA 3'end processing complex [GO:0071204] (cellular component) References: PMID:19470752 Sources: GOC:mah Definition: A ribonucleoprotein that binds to specific sites in, and is required for cleavage of, the 3'-end of histone pre-mRNAs. The complex contains the U7 snRNP and additional proteins, including the stem-loop binding protein (SLBP) and the exonuclease 3'hExo/Eri-1. Relationships: is a type of GO:0140513; is a type of ribonucleoprotein complex [GO:1990904] Also known as: histone 3'end pre-mRNA complex